{
  "gene_symbol": "MYCLP1",
  "gene_name": "Putative myc-like protein MYCLP1",
  "term_label": "Unknown cellular component",
  "gene": "UniProtKB:P12525",
  "term_id": "UNKNOWN:0003"
}